centromere localization [GO:0072765] (biological process) Also known as: establishment and maintenance of kinetochore localization, kinetochore localisation, kinetochore localization Sources: GOC:mah Subtypes: GO:0098653 Relationships: is a type of protein-containing complex localization [GO:0031503]; is a type of organelle localization [GO:0051640] Definition: A cellular localization process in which a centromere/kinetochore is transported to, or maintained in, a specific location.